{
  "gene_symbol": "PPARA",
  "term_label": "DNA-binding transcription repressor activity, RNA polymerase II-specific",
  "gene_name": "Peroxisome proliferator-activated receptor alpha",
  "term_id": "GO:0001227",
  "gene": "UniProtKB:Q07869"
}